{
  "gene": "UniProtKB:O00231",
  "term_label": "structural molecule activity",
  "term_id": "GO:0005198",
  "gene_name": "26S proteasome non-ATPase regulatory subunit 11",
  "gene_symbol": "PSMD11"
}